{
  "gene": "UniProtKB:Q5JRA6",
  "gene_symbol": "MIA3",
  "term_id": "GO:0070971",
  "gene_name": "Transport and Golgi organization protein 1 homolog",
  "term_label": "endoplasmic reticulum exit site"
}